{
  "gene_name": "General transcription factor II-I repeat domain-containing protein 2A",
  "gene": "UniProtKB:Q86UP8",
  "term_id": "UNKNOWN:0002",
  "gene_symbol": "GTF2IRD2",
  "term_label": "Unknown biological process"
}